thyroid hormone binding [GO:0070324] (molecular function) Definition: Binding to thyroxine (T4) or triiodothyronine (T3), tyrosine-based hormones produced by the thyroid gland. Sources: GOC:rph Relationships: is a type of GO:0042562 Also known as: thyroxine binding, triiodothyronine binding